{
  "term_id": "GO:0032874",
  "gene": "UniProtKB:Q7L7X3",
  "gene_symbol": "TAOK1",
  "gene_name": "Serine_threonine-protein kinase TAO1",
  "term_label": "positive regulation of stress-activated MAPK cascade"
}